{
  "gene": "UniProtKB:Q9HB07",
  "term_label": "Unknown molecular function",
  "gene_symbol": "MYG1",
  "gene_name": "MYG1 exonuclease",
  "term_id": "UNKNOWN:0001"
}